{
  "gene_symbol": "PLEC",
  "term_id": "GO:0005882",
  "term_label": "intermediate filament",
  "gene": "UniProtKB:Q15149",
  "gene_name": "Plectin"
}